{
  "gene": "UniProtKB:P51570",
  "term_label": "cytosol",
  "term_id": "GO:0005829",
  "gene_symbol": "GALK1",
  "gene_name": "Galactokinase"
}